{
  "gene_symbol": "SF3A2",
  "term_id": "GO:0071004",
  "gene": "UniProtKB:Q15428",
  "term_label": "U2-type prespliceosome",
  "gene_name": "Splicing factor 3A subunit 2"
}